{
  "gene": "UniProtKB:Q96LI6",
  "term_id": "GO:0003700",
  "term_label": "DNA-binding transcription factor activity",
  "gene_symbol": "HSFY2",
  "gene_name": "Heat shock transcription factor, Y-linked"
}